{
  "term_id": "GO:0048030",
  "gene_symbol": "LGALS3",
  "gene_name": "Galectin-3",
  "gene": "UniProtKB:P17931",
  "term_label": "disaccharide binding"
}